{
  "gene": "UniProtKB:A0A075B6V8",
  "gene_symbol": "TRAJ5",
  "gene_name": "T cell receptor alpha joining 5 (Fragment)",
  "term_label": "Unknown cellular component",
  "term_id": "UNKNOWN:0003"
}